regulation of membrane depolarization during AV node cell action potential [GO:1905027] (biological process) Relationships: is a type of regulation of AV node cell action potential [GO:0098904]; is a type of regulation of membrane depolarization during cardiac muscle cell action potential [GO:1900825]; regulates membrane depolarization during AV node cell action potential [GO:0086045] Subtypes: negative regulation of membrane depolarization during AV node cell action potential [GO:1905028], positive regulation of membrane depolarization during AV node cell action potential [GO:1905029] Definition: Any process that modulates the frequency, rate or extent of membrane depolarization during AV node cell action potential. Also known as: regulation of membrane depolarization during AV node cardiac muscle cell action potential, regulation of membrane depolarization during atrioventricular node cardiac muscle cell action potential References: PMID:19726871 Sources: GOC:BHF, GOC:BHF_miRNA, GOC:TermGenie, GOC:mtg_cardiac_conduct_nov11, GOC:rph